{
  "term_id": "GO:0005634",
  "term_label": "nucleus",
  "gene": "UniProtKB:Q9HCP0",
  "gene_symbol": "CSNK1G1",
  "gene_name": "Casein kinase I isoform gamma-1"
}